rhombomere 8 formation [GO:0021677] (biological process) Definition: The process that gives rise to rhombomere 8. This process pertains to the initial formation of a structure from unspecified parts. Rhombomeres are transverse segments of the developing rhombencephalon. Rhombomeres are lineage restricted, express different genes from one another, and adopt different developmental fates. Rhombomeres are numbered in anterior to posterior order. Relationships: is a type of rhombomere formation [GO:0021594]; is part of rhombomere 8 morphogenesis [GO:0021674] Sources: GOC:cls, GOC:curators, GOC:dgh, GOC:dph, GOC:jid